{
  "gene_name": "Protein Shroom4",
  "term_id": "GO:0007015",
  "gene_symbol": "SHROOM4",
  "term_label": "actin filament organization",
  "gene": "UniProtKB:Q9ULL8"
}